{
  "gene_name": "Semaphorin-3F",
  "term_id": "GO:0005886",
  "term_label": "plasma membrane",
  "gene": "UniProtKB:Q13275",
  "gene_symbol": "SEMA3F"
}